{
  "gene": "UniProtKB:Q9NPA2",
  "term_label": "plasma membrane",
  "gene_symbol": "MMP25",
  "term_id": "GO:0005886",
  "gene_name": "Matrix metalloproteinase-25"
}